{
  "gene_name": "Transmembrane protein 165",
  "term_id": "GO:0071421",
  "gene_symbol": "TMEM165",
  "term_label": "manganese ion transmembrane transport",
  "gene": "UniProtKB:Q9HC07"
}